{
  "term_label": "Unknown biological process",
  "gene_name": "UPF0688 protein C1orf174",
  "gene": "UniProtKB:Q8IYL3",
  "term_id": "UNKNOWN:0002",
  "gene_symbol": "C1orf174"
}